glial cell migration [GO:0008347] (biological process) Definition: The orderly movement of a glial cell, non-neuronal cells that provide support and nutrition, maintain homeostasis, form myelin, and participate in signal transmission in the nervous system. Sources: GOC:jl, GOC:mtg_sensu Relationships: is_a cell migration [GO:0016477]; is part of gliogenesis [GO:0042063] Also known as: glia cell migration Subtypes: telencephalon glial cell migration [GO:0022030], GO:0036135, astrocyte cell migration [GO:0043615], GO:0048896, GO:1904124 Regulation: regulated by regulation of glial cell migration [GO:1903975]; negatively regulated by negative regulation of glial cell migration [GO:1903976]; positively regulated by positive regulation of glial cell migration [GO:1903977]